{
  "term_id": "GO:0008331",
  "term_label": "high voltage-gated calcium channel activity",
  "gene_name": "Voltage-dependent T-type calcium channel subunit alpha-1G",
  "gene": "UniProtKB:O43497",
  "gene_symbol": "CACNA1G"
}